peptidoglycan-based cell wall [GO:0009274] (cellular component) Relationships: is_a cell wall [GO:0005618] Sources: GOC:mlg, ISBN:0815108893 Also known as: envelope, peptidoglycan, murein sacculus Subtypes: Gram-positive-bacterium-type cell wall [GO:0009275], Gram-negative-bacterium-type cell wall [GO:0009276] Definition: A protective structure outside the cytoplasmic membrane composed of peptidoglycan (also known as murein), a molecule made up of a glycan (sugar) backbone of repetitively alternating N-acetylglucosamine and N-acetylmuramic acid with short, attached, cross-linked peptide chains containing unusual amino acids. An example of this component is found in Escherichia coli.